establishment of mitochondrion localization by microtubule attachment [GO:0034640] (biological process) References: PMID:12972644 Sources: GOC:mah Relationships: is a type of GO:0034643; is a type of GO:0099098 Definition: The directed movement of a mitochondrion by attachment to a microtubule, followed by elongation of the microtubule by tubulin polymerization. Also known as: establishment of mitochondrion localisation by microtubule attachment, mitochondrial localization by microtubule attachment, mitochondrial migration by microtubule attachment, mitochondrion migration by microtubule attachment